apical plasma membrane urothelial plaque [GO:0120001] (cellular component) Relationships: is a type of plasma membrane [GO:0005886]; is_a GO:0098590; is part of apical plasma membrane [GO:0016324] References: PMID:21468280, PMID:21887288 Sources: GOC:krc Also known as: asymmetric unit membrane, AUM Definition: A scallop-shaped plaque, also referred to as an asymmetric unit membrane (AUM), found in the apical plasma membrane of urothelial superficial (umbrella) cells which form a a barrier to the passage of water and soluble toxic compounds found in urine. The plaques are thickened regions of membrane composed of uroplakin transmembrane proteins which form a crystalline array.